negative regulation of polyamine biosynthetic process [GO:0170066] (BP) References: PMID:9769097 Definition: Any process that stops, prevents, or reduces the frequency, rate or extent of polyamine biosynthesis. Polyamine biosynthesis is the chemical reactions and pathways resulting in the formation of polyamines, any organic compound containing two or more amino groups. Relationships: is_a GO:0009890; is a type of regulation of polyamine biosynthetic process [GO:0010967]; is a type of negative regulation of amine metabolic process [GO:0033239]; negatively regulates GO:0006596 Subtypes: GO:1901305